{
  "term_id": "GO:0030674",
  "term_label": "protein-macromolecule adaptor activity",
  "gene_name": "Male-specific lethal 1 homolog",
  "gene_symbol": "MSL1",
  "gene": "UniProtKB:Q68DK7"
}